N-acetylmannosamine biosynthetic process [GO:0006052] (biological process) Sources: GOC:ai, ISBN:0198506732 Relationships: is a type of N-acetylmannosamine metabolic process [GO:0006051]; is a type of mannosamine biosynthetic process [GO:0046347] Also known as: N-acetylmannosamine anabolism, N-acetylmannosamine biosynthesis, N-acetylmannosamine formation, N-acetylmannosamine synthesis Definition: The chemical reactions and pathways resulting in the formation of N-acetylmannosamine, the acetylated derivative of mannosamine, 2-amino-2-deoxymannose.